positive regulation of natural killer cell cytokine production [GO:0002729] (biological process) Definition: Any process that activates or increases the frequency, rate, or extent of natural killer cell cytokine production. Sources: GOC:add Also known as: positive regulation of NK cell cytokine production, up regulation of natural killer cell cytokine production, up-regulation of natural killer cell cytokine production, upregulation of natural killer cell cytokine production, activation of natural killer cell cytokine production, stimulation of natural killer cell cytokine production Relationships: is a type of positive regulation of natural killer cell mediated immunity [GO:0002717]; is a type of positive regulation of cytokine production involved in immune response [GO:0002720]; is a type of GO:0002727; positively regulates natural killer cell cytokine production [GO:0002370]